{
  "gene_symbol": "ID2",
  "gene": "UniProtKB:Q02363",
  "term_label": "negative regulation of transcription by RNA polymerase II",
  "gene_name": "DNA-binding protein inhibitor ID-2",
  "term_id": "GO:0000122"
}